{
  "term_label": "perineuronal net",
  "gene": "UniProtKB:Q96GW7",
  "term_id": "GO:0072534",
  "gene_symbol": "BCAN",
  "gene_name": "Brevican core protein"
}